cellular response to biotic stimulus [GO:0071216] (biological process) Subtypes: GO:0006983, cellular response to external biotic stimulus [GO:0071217], cellular response to molecule of bacterial origin [GO:0071219], GO:0071226, cellular response to molecule of oomycetes origin [GO:0071227], cellular response to tumor cell [GO:0071228], response to cell cycle checkpoint signaling [GO:0072396] Sources: GOC:mah Definition: Any process that results in a change in state or activity of a cell (in terms of movement, secretion, enzyme production, gene expression, etc.) as a result of a biotic stimulus, a stimulus caused or produced by a living organism. Also known as: cellular response to biotic stress Relationships: is a type of response to biotic stimulus [GO:0009607]; is a type of GO:0051716 Note: Note that this term is in the subset of terms that should not be used for direct gene product annotation. Instead, select a child term or, if no appropriate child term exists, please request a new term. Direct annotations to this term may be amended during annotation QC.